viral gene expression [GO:0019080] (biological process) Relationships: is a type of GO:0016032 Sources: GOC:bf, GOC:jl, ISBN:0121585336 Also known as: viral genome expression Definition: A process by which a viral gene is converted into a mature gene product or products (proteins or RNA). This includes viral transcription, processing to produce a mature RNA product, and viral translation.